{
  "term_id": "GO:0043083",
  "gene_name": "C1q-related factor",
  "gene": "UniProtKB:O75973",
  "term_label": "synaptic cleft",
  "gene_symbol": "C1QL1"
}